{
  "term_id": "UNKNOWN:0002",
  "gene": "UniProtKB:P0DV75",
  "gene_symbol": "FAM90A18",
  "gene_name": "Protein FAM90A18",
  "term_label": "Unknown biological process"
}